cartilage development [GO:0051216] (biological process) Regulation: regulated by regulation of cartilage development [GO:0061035]; positively regulated by positive regulation of cartilage development [GO:0061036]; negatively regulated by negative regulation of cartilage development [GO:0061037] Definition: The process whose specific outcome is the progression of a cartilage element over time, from its formation to the mature structure. Cartilage elements are skeletal elements that consist of connective tissue dominated by extracellular matrix containing collagen type II and large amounts of proteoglycan, particularly chondroitin sulfate. Also known as: cartilage biogenesis, cartilage biosynthesis, cartilage element development, cartilage formation, cartilage organ development, chondrogenesis Relationships: is_a animal organ development [GO:0048513]; is part of skeletal system development [GO:0001501]; is part of connective tissue development [GO:0061448] References: PMID:23251424 Sources: GOC:cjm Subtypes: cartilage development involved in endochondral bone morphogenesis [GO:0060351], bronchus cartilage development [GO:0060532], trachea cartilage development [GO:0060534], articular cartilage development [GO:0061975]